{
  "term_label": "glycosyltransferase activity",
  "gene_name": "Putative glycosyltransferase 6 domain-containing protein 1",
  "term_id": "GO:0016757",
  "gene_symbol": "GLT6D1",
  "gene": "UniProtKB:Q7Z4J2"
}